{
  "term_label": "membrane",
  "gene_name": "E3 ubiquitin-protein ligase HERC2",
  "term_id": "GO:0016020",
  "gene_symbol": "HERC2",
  "gene": "UniProtKB:O95714"
}